{
  "gene_symbol": "IL1F10",
  "gene_name": "Interleukin-1 family member 10",
  "gene": "UniProtKB:Q8WWZ1",
  "term_label": "cytokine-mediated signaling pathway",
  "term_id": "GO:0019221"
}